giant axon [GO:0042757] (cellular component) Relationships: is a type of GO:0030424 References: PMID:9705477 Sources: GOC:jl Definition: Extremely large, unmyelinated axon found in invertebrates. Has high conduction speeds and is usually involved in panic or escape responses.